gastric inhibitory peptide signaling pathway [GO:0038192] (biological process) Also known as: GIP signaling, gastric inhibitory polypeptide receptor signaling pathway, glucose-dependent insulinotropic polypeptide signaling Definition: A G protein-coupled receptor signaling pathway initiated by gastric inhibitory peptide (GIP) binding to its receptor on the surface of a target cell, and ending with the regulation of a downstream cellular process, e.g. transcription. Relationships: is a type of G protein-coupled receptor signaling pathway [GO:0007186] References: PMID:15955806 Sources: GOC:nhn